{
  "gene": "UniProtKB:Q96RG2",
  "gene_name": "PAS domain-containing serine_threonine-protein kinase",
  "gene_symbol": "PASK",
  "term_id": "GO:0035556",
  "term_label": "intracellular signal transduction"
}